{
  "gene_name": "Coronin-2A",
  "term_id": "GO:0005886",
  "gene": "UniProtKB:Q92828",
  "gene_symbol": "CORO2A",
  "term_label": "plasma membrane"
}